{
  "gene_name": "Zinc finger protein 816",
  "term_id": "GO:0000981",
  "gene": "UniProtKB:Q0VGE8",
  "term_label": "DNA-binding transcription factor activity, RNA polymerase II-specific",
  "gene_symbol": "ZNF816"
}